{
  "gene_name": "Homer protein homolog 3",
  "gene": "UniProtKB:Q9NSC5",
  "gene_symbol": "HOMER3",
  "term_label": "G protein-coupled glutamate receptor binding",
  "term_id": "GO:0035256"
}